{
  "gene": "UniProtKB:P35913",
  "term_id": "GO:0141162",
  "term_label": "negative regulation of cAMP/PKA signal transduction",
  "gene_symbol": "PDE6B",
  "gene_name": "Rod cGMP-specific 3',5'-cyclic phosphodiesterase subunit beta"
}